negative regulation of protein kinase activity [GO:0006469] (biological process) Also known as: down regulation of protein kinase activity, down-regulation of protein kinase activity, downregulation of protein kinase activity, inhibition of protein kinase activity Subtypes: negative regulation of protein kinase activity by regulation of protein phosphorylation [GO:0044387], negative regulation of protein tyrosine kinase activity [GO:0061099], negative regulation of protein serine/threonine kinase activity [GO:0071901], GO:1904030 Definition: Any process that stops, prevents, or reduces the frequency, rate or extent of protein kinase activity. Sources: GOC:go_curators Relationships: is a type of GO:0001933; is a type of GO:0033673; is a type of regulation of protein kinase activity [GO:0045859]; RO_0002212 protein kinase activity [GO:0004672]